{
  "term_id": "GO:0003729",
  "gene_name": "Putative testis-expressed protein 13C",
  "gene": "UniProtKB:A0A0J9YWL9",
  "term_label": "mRNA binding",
  "gene_symbol": "TEX13C"
}